positive regulation of metanephric DCT cell differentiation [GO:2000594] (biological process) Sources: GOC:obol Also known as: positive regulation of metanephric distal convoluted tubule cell differentiation Relationships: is_a positive regulation of cell differentiation [GO:0045597]; is_a regulation of metanephric DCT cell differentiation [GO:2000592]; positively regulates metanephric DCT cell differentiation [GO:0072240] Definition: Any process that activates or increases the frequency, rate or extent of metanephric DCT cell differentiation.